{
  "gene": "UniProtKB:Q8N6F7",
  "term_label": "regulation of B cell receptor signaling pathway",
  "gene_name": "Germinal center-associated signaling and motility protein",
  "term_id": "GO:0050855",
  "gene_symbol": "GCSAM"
}